cellular response to micafungin [GO:1903968] (biological process) Definition: Any process that results in a change in state or activity of a cell (in terms of movement, secretion, enzyme production, gene expression, etc.) as a result of a micafungin stimulus. References: PMID:16928959 Sources: GOC:TermGenie, GO_REF:0000071 Relationships: is a type of GO:0071396; is a type of cellular response to nitrogen compound [GO:1901699]; is a type of GO:1901701; is a type of response to micafungin [GO:1903967]